Ser(Gly)-tRNA(Ala) hydrolase activity [GO:0043908] (molecular function) References: PMID:14663147 Sources: GOC:jl Also known as: Ser(Gly)-tRNAAla hydrolase activity Definition: Catalysis of the hydrolysis of misacylated Ser-tRNA(Ala) and Gly-tRNA(Ala). Relationships: is a type of GO:0052689; is a type of catalytic activity, acting on a tRNA [GO:0140101]